positive regulation of chloroplast fission [GO:1905194] (biological process) Relationships: is a type of positive regulation of organelle organization [GO:0010638]; is a type of regulation of chloroplast fission [GO:1905192]; positively regulates chloroplast fission [GO:0010020] References: PMID:26862170 Sources: GOC:TermGenie, GO_REF:0000058 Note: Any process that modulates the rate, frequency or extent of chloroplast fission. Chloroplast fission is the division of a chloroplast within a cell to form two or more separate chloroplast compartments. Definition: Any process that activates or increases the frequency, rate or extent of chloroplast fission. Also known as: positive regulation of chloroplast division, up regulation of chloroplast division, up regulation of chloroplast fission, up-regulation of chloroplast division, up-regulation of chloroplast fission, upregulation of chloroplast division, upregulation of chloroplast fission, activation of chloroplast division, activation of chloroplast fission